positive regulation of mesenchymal cell apoptotic process [GO:2001055] (biological process) Definition: Any process that activates or increases the frequency, rate or extent of mesenchymal cell apoptotic process. Relationships: is a type of positive regulation of apoptotic process [GO:0043065]; is_a regulation of mesenchymal cell apoptotic process [GO:2001053]; RO_0002213 mesenchymal cell apoptotic process [GO:0097152] Sources: GOC:mtg_apoptosis, GOC:obol Also known as: positive regulation of mesenchymal cell apoptosis Subtypes: positive regulation of mesenchymal cell apoptotic process involved in nephron morphogenesis [GO:0072041], positive regulation of mesenchymal cell apoptotic process involved in metanephros development [GO:1900213]